{
  "term_label": "membrane",
  "term_id": "GO:0016020",
  "gene_symbol": "MTMR3",
  "gene": "UniProtKB:Q13615",
  "gene_name": "Myotubularin-related protein 3"
}